1,5-anhydro-D-fructose catabolic process [GO:1901802] (BP) Also known as: 1,5-anhydro-D-fructose breakdown, 1,5-anhydro-D-fructose catabolism, 1,5-anhydro-D-fructose degradation References: PMID:15716041 Sources: GOC:TermGenie, GOC:yaf, MetaCyc:PWY-6992, UniPathway:UPA00738 Definition: The chemical reactions and pathways resulting in the breakdown of 1,5-anhydro-D-fructose. Relationships: is_a ketone catabolic process [GO:0042182]; is a type of GO:0046174; is a type of monosaccharide catabolic process [GO:0046365]; is a type of epoxide metabolic process [GO:0097176]; is a type of ether catabolic process [GO:1901502]